GTPBP3-MTO1 complex [GO:7770010] (cellular component) References: PMID:29390138, PMID:33619562 Relationships: is a type of transferase complex [GO:1990234] Also known as: 5-taurinomethyluridine-tRNA synthase Definition: A protein complex consisting of GTP binding protein 3 (GTPBP3) and mitochondrial tRNA translation optimization 1 (MTO1). The complex catalyzes the formation of 5-taurinomethyluridine at wobble position U34 of mitochondrial tRNAs.